biotin biosynthetic process [GO:0009102] (biological process) Definition: The chemical reactions and pathways resulting in the formation of biotin, cis-tetrahydro-2-oxothieno(3,4-d)imidazoline-4-valeric acid. Also known as: biotin anabolism, biotin biosynthesis, biotin formation, biotin synthesis, vitamin B7 biosynthesis, vitamin B7 biosynthetic process, vitamin H biosynthesis, vitamin H biosynthetic process Relationships: is a type of biotin metabolic process [GO:0006768]; is a type of water-soluble vitamin biosynthetic process [GO:0042364]; is a type of GO:0043604; is a type of sulfur compound biosynthetic process [GO:0044272]; is a type of monocarboxylic acid biosynthetic process [GO:0072330] Sources: ISBN:0198506732